multiple spine synapse organization, single dendrite [GO:0150090] (biological process) Relationships: is a type of multiple spine synapse organization [GO:0150089] Definition: A process that is carried out at the cellular level which results in the assembly, arrangement of constituent parts, or disassembly of a synapse between a multiple synapse bouton and a single dendrite. References: PMID:10586883, PMID:11248111, PMID:22028887, PMID:24487234 Sources: GOC:aruk, GOC:bc